{
  "term_id": "GO:0001725",
  "gene_name": "Synaptopodin-2",
  "term_label": "stress fiber",
  "gene_symbol": "SYNPO2",
  "gene": "UniProtKB:Q9UMS6"
}